{
  "gene": "UniProtKB:O95751",
  "term_id": "UNKNOWN:0003",
  "gene_symbol": "LDOC1",
  "term_label": "Unknown cellular component",
  "gene_name": "Protein LDOC1"
}